negative regulation of nerve growth factor production [GO:0032904] (biological process) Definition: Any process that stops, prevents, or reduces the frequency, rate, or extent of production of nerve growth factor (NGF). Sources: GOC:mah Also known as: down regulation of nerve growth factor production, down-regulation of nerve growth factor production, downregulation of nerve growth factor production, negative regulation of NGF production, inhibition of nerve growth factor production Relationships: is a type of GO:0032900; is a type of GO:0032903; negatively regulates GO:0032902